{
  "gene_name": "Ubiquitin-like modifier-activating enzyme ATG7",
  "term_id": "GO:0019778",
  "term_label": "Atg12 activating enzyme activity",
  "gene_symbol": "ATG7",
  "gene": "UniProtKB:O95352"
}